{
  "gene_name": "Beta-defensin 104",
  "term_label": "innate immune response",
  "gene_symbol": "DEFB104A",
  "term_id": "GO:0045087",
  "gene": "UniProtKB:Q8WTQ1"
}